{
  "gene_symbol": "MTMR2",
  "term_label": "phosphatidylinositol-3,5-bisphosphate 3-phosphatase activity",
  "gene": "UniProtKB:Q13614",
  "gene_name": "Myotubularin-related protein 2",
  "term_id": "GO:0052629"
}